{
  "gene": "UniProtKB:Q8NA29",
  "term_id": "GO:0140329",
  "gene_symbol": "MFSD2A",
  "term_label": "lysophospholipid translocation",
  "gene_name": "Sodium-dependent lysophosphatidylcholine symporter 1"
}